{
  "term_id": "GO:0005829",
  "gene_symbol": "CRMP1",
  "gene": "UniProtKB:Q14194",
  "term_label": "cytosol",
  "gene_name": "Dihydropyrimidinase-related protein 1"
}